{
  "gene_symbol": "ODF2L",
  "gene": "UniProtKB:Q9ULJ1",
  "gene_name": "Protein BCAP",
  "term_label": "Unknown molecular function",
  "term_id": "UNKNOWN:0001"
}